ATP phosphoribosyltransferase activity [GO:0003879] (MF) Definition: Catalysis of the reaction: 1-(5-phospho-D-ribosyl)-ATP + diphosphate = ATP + 5-phospho-alpha-D-ribose 1-diphosphate. Relationships: is a type of pentosyltransferase activity [GO:0016763] Also known as: 1-(5-phospho-D-ribosyl)-ATP:diphosphate phospho-alpha-D-ribosyl-transferase activity, adenosine triphosphate phosphoribosyltransferase activity, phosphoribosyl ATP synthetase activity, phosphoribosyl ATP:pyrophosphate phosphoribosyltransferase activity, phosphoribosyl-ATP diphosphorylase activity, phosphoribosyl-ATP pyrophosphorylase activity, phosphoribosyl-ATP:pyrophosphate-phosphoribosyl phosphotransferase activity, phosphoribosyladenosine triphosphate pyrophosphorylase activity, phosphoribosyladenosine triphosphate synthetase activity, phosphoribosyladenosine triphosphate:pyrophosphate phosphoribosyltransferase activity Sources: EC:2.4.2.17